{
  "term_id": "GO:0001580",
  "gene": "UniProtKB:P59544",
  "term_label": "detection of chemical stimulus involved in sensory perception of bitter taste",
  "gene_name": "Taste receptor type 2 member 50",
  "gene_symbol": "TAS2R50"
}